{
  "term_label": "cilium assembly",
  "term_id": "GO:0060271",
  "gene_name": "Cytoplasmic dynein 2 heavy chain 1",
  "gene": "UniProtKB:Q8NCM8",
  "gene_symbol": "DYNC2H1"
}